{
  "gene_symbol": "TP53",
  "term_label": "promoter-specific chromatin binding",
  "term_id": "GO:1990841",
  "gene": "UniProtKB:P04637",
  "gene_name": "Cellular tumor antigen p53"
}